{
  "gene_symbol": "SLC2A6",
  "gene": "UniProtKB:Q9UGQ3",
  "gene_name": "Solute carrier family 2, facilitated glucose transporter member 6",
  "term_label": "membrane",
  "term_id": "GO:0016020"
}